{
  "term_id": "UNKNOWN:0003",
  "gene": "UniProtKB:Q86T75",
  "term_label": "Unknown cellular component",
  "gene_symbol": "NBPF11",
  "gene_name": "Neuroblastoma breakpoint family member 11"
}